polyamine catabolic process [GO:0006598] (biological process) Sources: ISBN:0198506732 Also known as: polyamine breakdown, polyamine catabolism, polyamine degradation Subtypes: GO:0009447, GO:0019381, spermidine catabolic process [GO:0046203], GO:0046205, spermine catabolic process [GO:0046208], trimethylenediamine catabolic process [GO:1901056], thermospermine catabolic process [GO:1903602] Definition: The chemical reactions and pathways resulting in the breakdown of polyamines, any organic compound containing two or more amino groups. Relationships: is a type of GO:0006595; is a type of biogenic amine catabolic process [GO:0042402]